{
  "gene_name": "Olfactory receptor 2J3",
  "term_id": "GO:0004984",
  "gene": "UniProtKB:O76001",
  "gene_symbol": "OR2J3",
  "term_label": "olfactory receptor activity"
}